{
  "term_id": "GO:0003823",
  "term_label": "antigen binding",
  "gene_name": "Immunoglobulin heavy variable 4-59",
  "gene": "UniProtKB:P01825",
  "gene_symbol": "IGHV4-59"
}